{
  "gene_name": "Complement receptor type 2",
  "gene": "UniProtKB:P20023",
  "gene_symbol": "CR2",
  "term_label": "negative regulation of complement activation, classical pathway",
  "term_id": "GO:0045959"
}